oxidoreductase activity, acting on a sulfur group of donors, oxygen as acceptor [GO:0016670] (molecular function) Also known as: oxidoreductase activity, acting on sulphur group of donors, oxygen as acceptor Definition: Catalysis of an oxidation-reduction (redox) reaction in which a sulfur-containing group acts as a hydrogen or electron donor and reduces oxygen. Relationships: is a type of oxidoreductase activity, acting on a sulfur group of donors [GO:0016667] Subtypes: prenylcysteine oxidase activity [GO:0001735], sulfite oxidase activity [GO:0008482], thiol oxidase activity [GO:0016972], methanethiol oxidase activity [GO:0018549], GO:0047950, GO:0102149, GO:0120147 Sources: GOC:jl